regulation of mitotic centrosome separation [GO:0046602] (biological process) Definition: Any process that modulates the frequency, rate or extent of the separation of duplicated centrosome components at the beginning of mitosis. Subtypes: negative regulation of mitotic centrosome separation [GO:0046603], positive regulation of mitotic centrosome separation [GO:0046604] Relationships: is a type of regulation of cell cycle process [GO:0010564]; regulates mitotic centrosome separation [GO:0007100] Sources: GOC:ai